fusome [GO:0045169] (cellular component) Definition: A large intracellular spectrin-rich structure that has been found in insect germline cells and mammalian hematopoietic cells. The fusome is an elongated, branched structure, formed from the spherical spectrosome organelle. Relationships: is a type of cellular anatomical structure [GO:0110165]; is part of cytoplasm [GO:0005737] References: PMID:12655376 Sources: GOC:bf